{
  "term_id": "GO:0030337",
  "term_label": "DNA polymerase processivity factor activity",
  "gene_symbol": "POLG2",
  "gene": "UniProtKB:Q9UHN1",
  "gene_name": "DNA polymerase subunit gamma-2, mitochondrial"
}